positive regulation of anterograde synaptic vesicle transport [GO:1903744] (biological process) Relationships: is a type of GO:1901610; is a type of GO:1902805; is a type of regulation of anterograde synaptic vesicle transport [GO:1903742]; positively regulates anterograde synaptic vesicle transport [GO:0048490] References: PMID:25329901 Sources: GOC:TermGenie, GOC:kmv, GO_REF:0000058 Definition: Any process that activates or increases the frequency, rate or extent of anterograde synaptic vesicle transport. Also known as: up regulation of anterograde synaptic vesicle transport, up-regulation of anterograde synaptic vesicle transport, upregulation of anterograde synaptic vesicle transport, activation of anterograde synaptic vesicle transport